{
  "gene_name": "Dual specificity protein phosphatase 22",
  "gene": "UniProtKB:Q9NRW4",
  "term_id": "GO:0007179",
  "term_label": "transforming growth factor beta receptor signaling pathway",
  "gene_symbol": "DUSP22"
}